{
  "term_label": "Unknown cellular component",
  "gene": "UniProtKB:Q8NGK9",
  "term_id": "UNKNOWN:0003",
  "gene_name": "Olfactory receptor 5D16",
  "gene_symbol": "OR5D16"
}